{
  "gene_symbol": "ZNF33A",
  "gene": "UniProtKB:Q06730",
  "gene_name": "Zinc finger protein 33A",
  "term_label": "transcription cis-regulatory region binding",
  "term_id": "GO:0000976"
}